{
  "term_id": "GO:0007416",
  "gene_symbol": "SDK2",
  "gene_name": "Protein sidekick-2",
  "term_label": "synapse assembly",
  "gene": "UniProtKB:Q58EX2"
}